{
  "term_label": "ATPase-coupled monoatomic cation transmembrane transporter activity",
  "gene": "UniProtKB:Q9HD20",
  "term_id": "GO:0019829",
  "gene_symbol": "ATP13A1",
  "gene_name": "Endoplasmic reticulum transmembrane helix translocase"
}